regulation of raffinose biosynthetic process [GO:1900091] (biological process) References: PMID:22307851 Sources: GOC:TermGenie Also known as: regulation of raffinose anabolism, regulation of raffinose biosynthesis, regulation of raffinose formation, regulation of raffinose synthesis Relationships: is a type of regulation of carbohydrate biosynthetic process [GO:0043255]; is a type of regulation of raffinose metabolic process [GO:0080091]; regulates raffinose biosynthetic process [GO:0033529] Subtypes: negative regulation of raffinose biosynthetic process [GO:1900092], GO:1900093 Definition: Any process that modulates the frequency, rate or extent of raffinose biosynthetic process.